{
  "term_id": "GO:0000077",
  "gene": "UniProtKB:Q8TEK3",
  "term_label": "DNA damage checkpoint signaling",
  "gene_name": "Histone-lysine N-methyltransferase, H3 lysine-79 specific",
  "gene_symbol": "DOT1L"
}